{
  "gene": "UniProtKB:P20340",
  "gene_symbol": "RAB6A",
  "term_id": "GO:0003924",
  "gene_name": "Ras-related protein Rab-6A",
  "term_label": "GTPase activity"
}